skeletal muscle fiber differentiation [GO:0098528] (biological process) Relationships: is a type of myotube differentiation [GO:0014902]; is a type of skeletal muscle cell differentiation [GO:0035914] Subtypes: tongue muscle cell differentiation [GO:0035981] Sources: GOC:dos Regulation: RO_0002211 by regulation of skeletal muscle fiber differentiation [GO:1902809]; negatively regulated by negative regulation of skeletal muscle fiber differentiation [GO:1902810]; positively regulated by GO:1902811 Definition: The process in which a relatively unspecialized cell acquires specialized features of a skeletal muscle fiber cell. Skeletal muscle fiber differentiation starts with myoblast fusion and the appearance of specific cell markers (this is the cell development step). Then individual skeletal muscle fibers fuse to form bigger myotubes and start to contract.